{
  "gene_symbol": "STAU2",
  "term_label": "germ cell development",
  "term_id": "GO:0007281",
  "gene": "UniProtKB:Q9NUL3",
  "gene_name": "Double-stranded RNA-binding protein Staufen homolog 2"
}